meiosis II cell cycle phase [GO:0098765] (biological process) Note: This term should not be used for direct annotation. If you are trying to make an annotation to x phase, it is likely that the correct annotation should be to 'regulation of x/y phase transition' or to a process which occurs during the reported phase (e.g. mitotic DNA replication for mitotic S-phase). To capture the phase when a specific location or process is observed, the phase term can be used in an annotation extension (PMID:24885854) applied to a cellular component term (with the relation exists_during) or a biological process term (with the relation happens_during). Relationships: is a type of meiotic cell cycle phase [GO:0098762] Definition: A meiotic cell cycle phase that occurs after meiosis I (the first meiotic nuclear division). Sources: GOC:dos Subtypes: meiotic prophase II [GO:0007136], GO:0007137, meiotic anaphase II [GO:0007138], GO:0007139, meiotic interphase II [GO:0044844]